methylmalonyl-CoA mutase activity [GO:0004494] (molecular function) Relationships: is a type of intramolecular transferase activity [GO:0016866] Also known as: (R)-2-methyl-3-oxopropanoyl-CoA CoA-carbonylmutase activity, (R)-methylmalonyl-CoA CoA-carbonylmutase activity, (S)-methylmalonyl-CoA mutase activity, methylmalonyl coenzyme A carbonylmutase activity, methylmalonyl coenzyme A mutase activity, methylmalonyl-CoA CoA-carbonyl mutase activity Definition: Catalysis of the reaction: (R)-methylmalonyl-CoA = succinyl-CoA. Sources: EC:5.4.99.2, RHEA:22888